{
  "gene": "UniProtKB:Q8NFY9",
  "term_label": "ubiquitin-like ligase-substrate adaptor activity",
  "gene_name": "Kelch repeat and BTB domain-containing protein 8",
  "gene_symbol": "KBTBD8",
  "term_id": "GO:1990756"
}